negative regulation of cellulose biosynthetic process [GO:2001007] (biological process) Sources: GOC:mengo_curators Also known as: negative regulation of cellulose anabolism, negative regulation of cellulose biosynthesis, negative regulation of cellulose formation, negative regulation of cellulose synthesis Subtypes: negative regulation of plant-type cell wall cellulose biosynthetic process [GO:2001010] Definition: Any process that stops, prevents or reduces the frequency, rate or extent of cellulose biosynthetic process. Relationships: is a type of negative regulation of macromolecule biosynthetic process [GO:0010558]; is_a GO:0045912; is a type of GO:2001006; negatively regulates cellulose biosynthetic process [GO:0030244]